{
  "term_id": "GO:0016925",
  "gene": "UniProtKB:Q9HCI6",
  "gene_name": "E3 SUMO-protein ligase KIAA1586",
  "gene_symbol": "KIAA1586",
  "term_label": "protein sumoylation"
}